maintenance of cell number [GO:0098727] (biological process) Subtypes: skeletal muscle satellite cell maintenance involved in skeletal muscle regeneration [GO:0014834], stem cell population maintenance [GO:0019827] Definition: Any process by which the numbers of cells of a particular type or in a tissue are maintained. Relationships: is a type of GO:0032502 Sources: GOC:dos